formation of specialized structure for nutrient acquisition [GO:0052093] (BP) Subtypes: GO:0052094, formation of syncytium involving giant cell for nutrient acquisition [GO:0052096], formation of arbuscule for nutrient acquisition [GO:0075328], formation of stylet for nutrient acquisition [GO:0085001], formation of tubovesicular network for nutrient acquisition [GO:0085019] Also known as: formation by organism of specialized structure for nutrient acquisition from host, formation by symbiont of specialized structure for nutrient acquisition from host, formation of specialized structure for nutrient acquisition from host Sources: GOC:mtg_pamgo_17jul06 Relationships: is a type of formation of structure involved in a symbiotic process [GO:0044111]; is part of acquisition of nutrients from host [GO:0044002] Definition: The assembly of a symbiotic cellular or anatomical structure for the purpose of obtaining nutrients from its host organism. The host is defined as the larger of the organisms involved in a symbiotic interaction.